{
  "term_id": "GO:0019005",
  "gene": "UniProtKB:Q13616",
  "gene_name": "Cullin-1",
  "gene_symbol": "CUL1",
  "term_label": "SCF ubiquitin ligase complex"
}